{
  "gene_name": "Probable mitochondrial glutathione transporter SLC25A40",
  "term_id": "UNKNOWN:0002",
  "term_label": "Unknown biological process",
  "gene": "UniProtKB:Q8TBP6",
  "gene_symbol": "SLC25A40"
}